{
  "term_label": "ubiquitin protein ligase binding",
  "gene": "UniProtKB:Q8IVM0",
  "gene_symbol": "CCDC50",
  "gene_name": "Coiled-coil domain-containing protein 50",
  "term_id": "GO:0031625"
}